{
  "term_label": "centrosome",
  "term_id": "GO:0005813",
  "gene": "UniProtKB:O94927",
  "gene_symbol": "HAUS5",
  "gene_name": "HAUS augmin-like complex subunit 5"
}